{
  "term_label": "DNA-binding transcription factor activity",
  "term_id": "GO:0003700",
  "gene_symbol": "BCL11B",
  "gene": "UniProtKB:Q9C0K0",
  "gene_name": "B-cell lymphoma_leukemia 11B"
}